{
  "term_id": "GO:0005634",
  "term_label": "nucleus",
  "gene_name": "Zinc finger protein 69 homolog",
  "gene_symbol": "ZFP69",
  "gene": "UniProtKB:Q49AA0"
}